{
  "gene_symbol": "USP38",
  "gene_name": "Ubiquitin carboxyl-terminal hydrolase 38",
  "term_label": "regulation of protein stability",
  "term_id": "GO:0031647",
  "gene": "UniProtKB:Q8NB14"
}